ureidosuccinase activity [GO:0050386] (molecular function) Relationships: is a type of hydrolase activity, acting on carbon-nitrogen (but not peptide) bonds, in linear amides [GO:0016811] Also known as: N-carbamoyl-L-aspartate amidohydrolase activity Sources: EC:3.5.1.7, RHEA:14365 Definition: Catalysis of the reaction: N-carbamoyl-L-aspartate + H2O + 2 H+ = L-aspartate + CO2 + NH4.